{
  "term_label": "Unknown biological process",
  "gene_symbol": "CD302",
  "term_id": "UNKNOWN:0002",
  "gene": "UniProtKB:Q8IX05",
  "gene_name": "CD302 antigen"
}